auxin-activated signaling pathway [GO:0009734] (biological process) Definition: The series of molecular signals generated by the binding of the plant hormone auxin to a receptor, and ending with modulation of a downstream cellular process, e.g. transcription. References: PMID:16990790, PMID:18647826 Sources: GOC:mah, GOC:sm Also known as: auxin mediated signalling, auxin signal transduction, auxin signaling, auxin mediated signaling pathway, auxin-regulated transcription Relationships: is a type of hormone-mediated signaling pathway [GO:0009755]; is part of cellular response to auxin stimulus [GO:0071365] Subtypes: positive regulation of leaflet formation by auxin mediated signaling pathway [GO:0090015] Regulation: regulated by regulation of auxin mediated signaling pathway [GO:0010928]; positively regulated by GO:0010929; negatively regulated by negative regulation of auxin mediated signaling pathway [GO:0010930]